{
  "gene": "UniProtKB:Q9Y520",
  "gene_name": "Protein PRRC2C",
  "term_id": "UNKNOWN:0001",
  "term_label": "Unknown molecular function",
  "gene_symbol": "PRRC2C"
}